lung saccule development [GO:0060430] (biological process) Relationships: is a type of GO:0048856; BFO_0000050 lung alveolus development [GO:0048286] Definition: The biological process whose specific outcome is the progression of a lung saccule from an initial condition to its mature state. The lung saccule is the primitive gas exchange portion of the lung composed of type I and type II cells. Also known as: lung saccular development Sources: GOC:dph, GOC:mtg_lung